negative regulation of autophagy of mitochondrion [GO:1903147] (biological process) References: PMID:24600391 Sources: GOC:PARL, GOC:TermGenie, GOC:autophagy, GOC:bf, GO_REF:0000058 Relationships: is_a negative regulation of autophagy [GO:0010507]; is_a regulation of autophagy of mitochondrion [GO:1903146]; negatively regulates autophagy of mitochondrion [GO:0000422] Definition: Any process that stops, prevents or reduces the frequency, rate or extent of mitochondrion degradation by autophagy. Also known as: down regulation of mitochondrial degradation, down regulation of mitochondrion degradation, down-regulation of mitochondrion degradation, down-regulation of mitophagy, downregulation of mitochondrion degradation, inhibition of mitophagy, inhibition of mitochondrion degradation Subtypes: negative regulation of mitophagy [GO:1901525]